{
  "term_label": "olfactory receptor activity",
  "gene_name": "Olfactory receptor 6Q1",
  "term_id": "GO:0004984",
  "gene_symbol": "OR6Q1",
  "gene": "UniProtKB:Q8NGQ2"
}